regulation of microtubule anchoring at centrosome [GO:0150101] (biological process) Relationships: is a type of regulation of microtubule cytoskeleton organization [GO:0070507]; regulates microtubule anchoring at centrosome [GO:0034454] Definition: Any process that modulates the frequency, rate or extent of microtubule anchoring at centrosome. References: PMID:17139249 Sources: GOC:aruk, GOC:bc